proplastid [GO:0009537] (cellular component) Definition: The precursor of other plastids. Relationships: is a type of plastid [GO:0009536] Sources: ISBN:0943088399